{
  "gene_name": "Putative zinc finger protein 542",
  "term_label": "Unknown biological process",
  "gene": "UniProtKB:Q5EBM4",
  "gene_symbol": "ZNF542P",
  "term_id": "UNKNOWN:0002"
}